T=25 icosahedral viral capsid [GO:0039623] (cellular component) Definition: The protein coat that surrounds the infective nucleic acid in some virus particles where the subunits (capsomeres) are arranged to form an icosahedron with T=25 symmetry. The T=25 capsid is composed of 12 pentameric and 240 hexameric capsomeres. Sources: VZ:810 Relationships: is a type of icosahedral viral capsid [GO:0019030]